{
  "term_label": "postsynaptic density membrane",
  "term_id": "GO:0098839",
  "gene_symbol": "GRID2",
  "gene_name": "Glutamate receptor ionotropic, delta-2",
  "gene": "UniProtKB:O43424"
}